{
  "gene_name": "GTP-binding nuclear protein Ran",
  "term_id": "GO:0005634",
  "gene": "UniProtKB:P62826",
  "term_label": "nucleus",
  "gene_symbol": "RAN"
}